{
  "gene_symbol": "CTLA4",
  "gene": "UniProtKB:P16410",
  "gene_name": "Cytotoxic T-lymphocyte protein 4",
  "term_label": "external side of plasma membrane",
  "term_id": "GO:0009897"
}